{
  "term_id": "GO:0000981",
  "gene": "UniProtKB:O14978",
  "gene_name": "Zinc finger protein 263",
  "term_label": "DNA-binding transcription factor activity, RNA polymerase II-specific",
  "gene_symbol": "ZNF263"
}